{
  "term_label": "phospholipase activity",
  "term_id": "GO:0004620",
  "gene": "UniProtKB:O94830",
  "gene_symbol": "DDHD2",
  "gene_name": "Phospholipase DDHD2"
}